{
  "gene": "UniProtKB:Q9NQU5",
  "term_id": "GO:0043408",
  "gene_name": "Serine_threonine-protein kinase PAK 6",
  "term_label": "regulation of MAPK cascade",
  "gene_symbol": "PAK6"
}